{
  "gene_symbol": "MRPL58",
  "gene_name": "Large ribosomal subunit protein mL62",
  "term_label": "mitochondrial translational termination",
  "gene": "UniProtKB:Q14197",
  "term_id": "GO:0070126"
}